{
  "gene_name": "Retinoic acid receptor responder protein 2",
  "gene_symbol": "RARRES2",
  "term_id": "GO:0050921",
  "term_label": "positive regulation of chemotaxis",
  "gene": "UniProtKB:Q99969"
}